{
  "gene_name": "Ketosamine-3-kinase",
  "term_id": "UNKNOWN:0002",
  "gene": "UniProtKB:Q9HA64",
  "term_label": "Unknown biological process",
  "gene_symbol": "FN3KRP"
}